{
  "gene_symbol": "SMARCD1",
  "term_label": "transcription coregulator activity",
  "term_id": "GO:0003712",
  "gene": "UniProtKB:Q96GM5",
  "gene_name": "SWI_SNF-related matrix-associated actin-dependent regulator of chromatin subfamily D member 1"
}